{
  "term_label": "Unknown biological process",
  "gene_symbol": "GPA33",
  "term_id": "UNKNOWN:0002",
  "gene_name": "Cell surface A33 antigen",
  "gene": "UniProtKB:Q99795"
}